1-phosphatidylinositol-5-phosphate 4-kinase activity [GO:0016309] (molecular function) Relationships: is a type of phosphatidylinositol kinase activity [GO:0052742] Sources: EC:2.7.1.149 Also known as: 1-phosphatidylinositol-5-phosphate kinase, PIP4K, type II PIP kinase activity, ATP:1-phosphatidyl-1D-myo-inositol-5-phosphate 4-phosphotransferase activity Definition: Catalysis of the reaction: a 1-phosphatidyl-1D-myo-inositol 5-phosphate + ATP = a 1-phosphatidyl-1D-myo-inositol 4,5-bisphosphate + ADP + H+.